{
  "gene_name": "Centrosome and spindle pole-associated protein 1",
  "gene_symbol": "CSPP1",
  "gene": "UniProtKB:Q1MSJ5",
  "term_label": "centrosome",
  "term_id": "GO:0005813"
}